{
  "term_id": "GO:0008970",
  "gene": "UniProtKB:Q9Y5X9",
  "gene_symbol": "LIPG",
  "term_label": "phospholipase A1 activity",
  "gene_name": "Endothelial lipase"
}